biotin metabolic process [GO:0006768] (biological process) Definition: The chemical reactions and pathways involving biotin, cis-tetrahydro-2-oxothieno(3,4-d)imidazoline-4-valeric acid; the (+) enantiomer is very widely distributed in cells and serves as a carrier in a number of enzymatic beta-carboxylation reactions. Relationships: is a type of sulfur compound metabolic process [GO:0006790]; is a type of monocarboxylic acid metabolic process [GO:0032787]; is a type of amide metabolic process [GO:0043603] Sources: ISBN:0198506732 Subtypes: biotin biosynthetic process [GO:0009102], biotin catabolic process [GO:0042367] Also known as: biotin metabolism, vitamin B7 metabolic process, vitamin B7 metabolism, vitamin H metabolic process, vitamin H metabolism